{
  "gene_symbol": "CHRNA3",
  "term_id": "GO:0045202",
  "gene": "UniProtKB:P32297",
  "term_label": "synapse",
  "gene_name": "Neuronal acetylcholine receptor subunit alpha-3"
}